{
  "term_label": "mRNA binding",
  "term_id": "GO:0003729",
  "gene_name": "KH domain-containing RNA-binding protein QKI",
  "gene_symbol": "QKI",
  "gene": "UniProtKB:Q96PU8"
}